{
  "gene_symbol": "A8MVJ9",
  "gene_name": "Putative histone PARylation factor 1-like",
  "term_label": "poly-ADP-D-ribose binding",
  "term_id": "GO:0072572",
  "gene": "UniProtKB:A8MVJ9"
}